mitochondrial protein catabolic process [GO:0035694] (biological process) Also known as: catabolism of mitochondrial protein, degradation of damaged mitochondrial protein Definition: The chemical reactions and pathways resulting in the breakdown of a mitochondrial protein. This process is necessary to maintain the healthy state of mitochondria and is thought to occur via the induction of an intramitochondrial lysosome-like organelle that acts to eliminate the damaged oxidised mitochondrial proteins without destroying the mitochondrial structure. Relationships: is a type of protein catabolic process [GO:0030163]; is part of GO:0007005; occurs in mitochondrion [GO:0005739] References: PMID:21264221, PMID:21264228 Sources: GOC:sp